alliin lyase activity [GO:0047654] (molecular function) Sources: EC:4.4.1.4, MetaCyc:ALLIIN-LYASE-RXN Also known as: L-cysteine sulfoxide lyase activity, S-alkyl-L-cysteine S-oxide alkyl-sulfenate-lyase (2-aminoacrylate-forming), S-alkylcysteine sulfoxide lyase activity, alkylcysteine sulfoxide lyase activity, alliin alkyl-sulfenate-lyase activity, alliinase activity, cysteine sulfoxide lyase activity, cysteine sulphoxide lyase activity Relationships: is a type of carbon-sulfur lyase activity [GO:0016846] Definition: Catalysis of the reaction: an S-alkyl-L-cysteine S-oxide = an alkyl sulfenate + 2-aminoacrylate.